{
  "term_label": "nucleoplasm",
  "gene_symbol": "TRMT10B",
  "gene": "UniProtKB:Q6PF06",
  "gene_name": "tRNA methyltransferase 10 homolog B",
  "term_id": "GO:0005654"
}